{
  "term_id": "UNKNOWN:0001",
  "term_label": "Unknown molecular function",
  "gene_symbol": "NPIPB2",
  "gene": "UniProtKB:A6NJ64",
  "gene_name": "Putative nuclear pore complex-interacting protein family member B2"
}